cysteine-glucosaminylinositol ligase activity [GO:0035446] (molecular function) Relationships: is a type of acid-ammonia (or amide) ligase activity [GO:0016880] Definition: Catalysis of the reaction: 1-(2-amino-2-deoxy-alpha-D-glucopyranoside)-1D-myo-inositol + L-cysteine + ATP = 1-D-myo-inosityl-2-L-cysteinylamido-2-deoxy-alpha-D-glucopyranoside + AMP + diphosphate + 2 H+. 1-(2-amino-2-deoxy-alpha-D-glucopyranoside)-1D-myo-inositol is also known as glucosaminyl-inositol or GlcN-Ins, and 1-D-myo-inosityl-2-L-cysteinylamido-2-deoxy-alpha-D-glucopyranoside as desacetylmycothiol or Cys-GlcN-Ins. References: PMID:12033919 Sources: EC:6.3.1.13 Also known as: L-cysteine:1D-myo-inositol 2-amino-2-deoxy-alpha-D-glucopyranoside ligase, MshC ligase, desacetylmycothiol synthase